{
  "gene_name": "Lysosomal thioesterase PPT2",
  "term_id": "GO:0005576",
  "term_label": "extracellular region",
  "gene": "UniProtKB:Q9UMR5",
  "gene_symbol": "PPT2"
}